DNA-dependent protein kinase activity [GO:0004677] (molecular function) Note: This reaction requires the presence of DNA. Sources: GOC:mah Relationships: is a type of protein serine/threonine kinase activity [GO:0004674] Definition: DNA dependent catalysis of the reaction: ATP + a protein = ADP + a phosphoprotein.